{
  "gene": "UniProtKB:Q8NFH5",
  "gene_symbol": "NUP35",
  "term_id": "GO:0017056",
  "term_label": "structural constituent of nuclear pore",
  "gene_name": "Nucleoporin NUP35"
}